{
  "gene_name": "Enolase-phosphatase E1",
  "term_label": "Unknown cellular component",
  "term_id": "UNKNOWN:0003",
  "gene": "UniProtKB:Q9UHY7",
  "gene_symbol": "ENOPH1"
}